{
  "gene_symbol": "MINAR2",
  "gene_name": "Major intrinsically disordered NOTCH2-binding receptor 1-like",
  "gene": "UniProtKB:P59773",
  "term_id": "UNKNOWN:0001",
  "term_label": "Unknown molecular function"
}